{
  "term_id": "GO:0140206",
  "gene": "UniProtKB:P46059",
  "term_label": "dipeptide import across plasma membrane",
  "gene_name": "Solute carrier family 15 member 1",
  "gene_symbol": "SLC15A1"
}